NEDD8 transferase activity [GO:0019788] (molecular function) Relationships: is a type of ubiquitin-like protein transferase activity [GO:0019787] Definition: Catalysis of the transfer of NEDD8 from one protein to another via the reaction X-NEDD8 + Y = Y-NEDD8 + X, where both X-NEDD8 and Y-NEDD8 are covalent linkages. Sources: GOC:mah Also known as: Hub1 conjugating enzyme activity, NEDD8 conjugating enzyme activity, RUB1 conjugating enzyme activity Subtypes: NEDD8 conjugating enzyme activity [GO:0061654], NEDD8 ligase activity [GO:0061663]